{
  "gene_name": "Probable E3 ubiquitin-protein ligase HECTD4",
  "gene_symbol": "HECTD4",
  "gene": "UniProtKB:Q9Y4D8",
  "term_id": "GO:0042593",
  "term_label": "glucose homeostasis"
}